negative regulation of fibroblast apoptotic process [GO:2000270] (biological process) Definition: Any process that stops, prevents or reduces the frequency, rate or extent of fibroblast apoptotic process. Sources: GOC:mtg_apoptosis, GOC:obol, GOC:yaf Also known as: negative regulation of fibroblast apoptosis Relationships: is a type of negative regulation of apoptotic process [GO:0043066]; is a type of GO:2000269; negatively regulates fibroblast apoptotic process [GO:0044346]